{
  "term_id": "GO:0005125",
  "gene": "UniProtKB:O95150",
  "gene_name": "Tumor necrosis factor ligand superfamily member 15",
  "gene_symbol": "TNFSF15",
  "term_label": "cytokine activity"
}